negative regulation of protein localization to endosome [GO:1905667] (biological process) Definition: Any process that stops, prevents or reduces the frequency, rate or extent of protein localization to endosome. References: PMID:22732145 Sources: GOC:PARL, GOC:TermGenie, GOC:bc, GO_REF:0000058 Relationships: is a type of GO:1903828; is_a GO:1905666; negatively regulates GO:0036010 Also known as: down regulation of protein localisation in endosome, down regulation of protein localization in endosome, down regulation of protein localization to endosome, down-regulation of protein localisation in endosome, down-regulation of protein localization in endosome, down-regulation of protein localization to endosome, downregulation of protein localisation in endosome, downregulation of protein localization in endosome, downregulation of protein localization to endosome, negative regulation of protein localisation in endosome, negative regulation of protein localization in endosome, inhibition of protein localisation in endosome, inhibition of protein localization in endosome, inhibition of protein localization to endosome